{
  "term_id": "GO:0005549",
  "gene_symbol": "OR8G2P",
  "gene_name": "Putative olfactory receptor 8G2",
  "gene": "UniProtKB:Q6IF36",
  "term_label": "odorant binding"
}